replicative senescence [GO:0090399] (biological process) Definition: The process by which normal somatic cells reach an irreversible stage of cell cycle arrest following multiple rounds of replication; this end stage is associated with marked changes in gene expression and function. This is a natural barrier to unlimited proliferation of somatic cells, and is believed to be contolled by telomere shortening. Regulation: regulated by regulation of replicative senescence [GO:1904726]; negatively regulated by negative regulation of replicative senescence [GO:1904727]; positively regulated by positive regulation of replicative senescence [GO:1904728] References: PMID:17014937, PMID:23061726 Relationships: is a type of cell cycle process [GO:0022402]